negative regulation of p38MAPK cascade [GO:1903753] (biological process) Also known as: down regulation of p38 MAPK cascade, down regulation of p38 cascade, down regulation of p38MAPK cascade, down-regulation of p38 MAPK cascade, down-regulation of p38 cascade, down-regulation of p38MAPK cascade, downregulation of p38 MAPK cascade, downregulation of p38 cascade, downregulation of p38MAPK cascade, negative regulation of p38 MAPK cascade, negative regulation of p38 cascade, inhibition of p38 MAPK cascade, inhibition of p38 cascade, inhibition of p38MAPK cascade, negative regulation of osmosensory signaling MAPK cascade References: PMID:18681888 Sources: GOC:TermGenie, GO_REF:0000058 Definition: Any process that stops, prevents or reduces the frequency, rate or extent of p38MAPK cascade. Relationships: is a type of negative regulation of MAPK cascade [GO:0043409]; is a type of regulation of p38MAPK cascade [GO:1900744]; negatively regulates p38MAPK cascade [GO:0038066]